{
  "gene_symbol": "GAS6",
  "gene": "UniProtKB:Q14393",
  "term_label": "negative regulation of apoptotic process",
  "term_id": "GO:0043066",
  "gene_name": "Growth arrest-specific protein 6"
}